{
  "term_label": "calcium ion binding",
  "gene_symbol": "CASQ2",
  "gene_name": "Calsequestrin-2",
  "term_id": "GO:0005509",
  "gene": "UniProtKB:O14958"
}